{
  "term_label": "Unknown cellular component",
  "gene_name": "Paired box protein Pax-8",
  "term_id": "UNKNOWN:0003",
  "gene_symbol": "PAX8",
  "gene": "UniProtKB:Q06710"
}